optic nerve structural organization [GO:0021633] (biological process) Relationships: is a type of GO:0021604; is part of optic nerve morphogenesis [GO:0021631] Definition: The process that contributes to the act of creating the structural organization of the optic nerve. This process pertains to the physical shaping of a rudimentary structure. The sensory optic nerve originates from the bipolar cells of the retina and conducts visual information to the brainstem. The optic nerve exits the back of the eye in the orbit, enters the optic canal, and enters the central nervous system at the optic chiasm (crossing) where the nerve fibers become the optic tract just prior to entering the hindbrain. Also known as: optic nerve structural organisation, CN II structural organization Sources: GOC:cls, GOC:dgh, GOC:dph, GOC:jid, GO_REF:0000021